{
  "term_label": "Unknown molecular function",
  "term_id": "UNKNOWN:0001",
  "gene_symbol": "C8orf82",
  "gene": "UniProtKB:Q6P1X6",
  "gene_name": "UPF0598 protein C8orf82"
}